{
  "term_label": "nuclear import signal receptor activity",
  "term_id": "GO:0061608",
  "gene_symbol": "NUTF2",
  "gene": "UniProtKB:P61970",
  "gene_name": "Nuclear transport factor 2"
}